regulation of mononuclear cell migration [GO:0071675] (biological process) Sources: GOC:mah Definition: Any process that modulates the rate, frequency or extent of mononuclear cell migration. Mononuclear cell migration is the movement of a mononuclear cell within or between different tissues and organs of the body. Subtypes: GO:0071676, GO:0071677, regulation of monocyte chemotaxis [GO:0090025], regulation of macrophage migration [GO:1905521], GO:2000401, regulation of monocyte extravasation [GO:2000437], regulation of dendritic cell chemotaxis [GO:2000508] Relationships: is_a regulation of leukocyte migration [GO:0002685]; RO_0002211 mononuclear cell migration [GO:0071674]